nicotinate N-methyltransferase activity [GO:0008938] (molecular function) Relationships: is a type of GO:0008170; is a type of S-adenosylmethionine-dependent methyltransferase activity [GO:0008757] Sources: EC:2.1.1.7, RHEA:20241 Also known as: S-adenosyl-L-methionine:nicotinate N-methyltransferase activity, furanocoumarin 8-O-methyltransferase activity Definition: Catalysis of the reaction: S-adenosyl-L-methionine(1+) + nicotinate = N-methylnicotinate + S-adenosyl-L-homocysteine.